inositol-polyphosphate 5-phosphatase activity [GO:0004445] (molecular function) Also known as: L-myo-inositol 1,4,5-trisphosphate-monoesterase activity, inositol 1,4,5-trisphosphate phosphatase activity, inositol phosphate 5-phosphomonoesterase activity, 1D-myo-inositol-1,4,5-trisphosphate 5-phosphohydrolase activity, D-myo-inositol 1,4,5-triphosphate 5-phosphatase activity, D-myo-inositol 1,4,5-trisphosphate 5-phosphatase activity, Ins(1,4,5)P(3) 5-phosphatase activity, Ins(1,4,5)P3 5-phosphatase activity, InsP(3)/Ins(1,3,4,5)P(4) 5-phosphatase activity, InsP3/Ins(1,3,4,5)P4 5-phosphatase activity, inositol-1,4,5-trisphosphate 5-phosphatase activity, myo-inositol-1,4,5-trisphosphate 5-phosphatase activity, type II inositol-1,4,5-trisphosphate 5-phosphatase activity, 5PTase activity, D-myo-inositol(1,4,5)/(1,3,4,5)-polyphosphate 5-phosphatase activity, Ins(1,4,5)P3/Ins(1,3,4,5)P4 5-phosphatase activity, inosine triphosphatase activity, inositol polyphosphate-5-phosphatase activity, inositol triphosphate 5-phosphomonoesterase activity, inositol trisphosphate phosphomonoesterase activity, inositol-1,4,5-trisphosphate/1,3,4,5-tetrakisphosphate 5-phosphatase activity, type I inositol-polyphosphate phosphatase activity, type II inositol polyphosphate 5-phosphatase activity Sources: EC:3.1.3.56 Definition: Catalysis of the reactions: D-myo-inositol 1,4,5-trisphosphate + H2O = myo-inositol 1,4-bisphosphate + phosphate, and 1D-myo-inositol 1,3,4,5-tetrakisphosphate + H2O = 1D-myo-inositol 1,3,4-trisphosphate + phosphate. Note: Note that this is a compound function and should be replaced by 'GO:0052659 : inositol 1,3,4,5-tetrakisphosphate 5-phosphatase activity' and 'GO:0052658 : inositol-1,4,5-trisphosphate 5-phosphatase activity'. Relationships: is a type of inositol trisphosphate phosphatase activity [GO:0046030] Subtypes: inositol-1,4,5-trisphosphate 5-phosphatase activity [GO:0052658], GO:0052659